{
  "term_id": "UNKNOWN:0001",
  "gene": "UniProtKB:Q569K6",
  "gene_name": "Coiled-coil domain-containing protein 157",
  "term_label": "Unknown molecular function",
  "gene_symbol": "CCDC157"
}